{
  "gene_name": "ER membrane protein complex subunit 2",
  "term_id": "GO:0032977",
  "term_label": "membrane insertase activity",
  "gene_symbol": "EMC2",
  "gene": "UniProtKB:Q15006"
}